response to UV-B [GO:0010224] (biological process) Subtypes: cellular response to UV-B [GO:0071493] Also known as: response to UV-B light stimulus, response to UV-B radiation stimulus, response to UVB light stimulus, response to UVB radiation stimulus, response to medium wave ultraviolet light stimulus, response to medium wave ultraviolet radiation stimulus Definition: Any process that results in a change in state or activity of a cell or an organism (in terms of movement, secretion, enzyme production, gene expression, etc.) as a result of a UV-B radiation stimulus. UV-B radiation (UV-B light) spans the wavelengths 280 to 315 nm. Sources: GOC:tb Relationships: is a type of response to UV [GO:0009411]